mesonephric glomerular mesangial cell fate commitment [GO:0061264] (biological process) Sources: GOC:mtg_kidney_jan10 Relationships: is a type of glomerular mesangial cell fate commitment [GO:0072152]; is part of mesonephric glomerular mesangial cell differentiation [GO:0061259] Definition: The process in which the developmental fate of a cell becomes restricted such that it will develop into a mesonephric glomerular mesangial cell.